ATP-dependent activity, acting on DNA [GO:0008094] (molecular function) Also known as: ATPase activity, acting on DNA, ATPase, acting on DNA, DNA dependent ATPase activity, DNA-dependent ATPase activity, DNA-dependent adenosinetriphosphatase activity, adenosinetriphosphatase (DNA-dependent) Sources: GOC:pdt Relationships: is a type of catalytic activity, acting on DNA [GO:0140097]; is a type of ATP-dependent activity [GO:0140657] Definition: Catalytic activity that acts to modify DNA, driven by ATP hydrolysis. Subtypes: GO:0003678, DNA clamp loader activity [GO:0003689], DNA topoisomerase type II (double strand cut, ATP-hydrolyzing) activity [GO:0003918], DNA translocase activity [GO:0015616], DNA/RNA helicase activity [GO:0033677], GO:0036310, DNA clamp unloader activity [GO:0061860], GO:0120328, ATP-dependent protein-DNA unloader activity [GO:0140083], ATP-dependent chromatin remodeler activity [GO:0140658], ATP-dependent DNA damage sensor activity [GO:0140664]